{
  "term_id": "UNKNOWN:0002",
  "gene_name": "Olfactory receptor 5K3",
  "gene": "UniProtKB:A6NET4",
  "term_label": "Unknown biological process",
  "gene_symbol": "OR5K3"
}